{
  "gene": "UniProtKB:Q15185",
  "gene_symbol": "PTGES3",
  "term_label": "Hsp90 protein binding",
  "gene_name": "Prostaglandin E synthase 3",
  "term_id": "GO:0051879"
}